pseudocleavage [GO:0030588] (biological process) Subtypes: pseudocleavage involved in syncytial blastoderm formation [GO:0030589], first cell cycle pseudocleavage [GO:0030590] Definition: Partial constriction of the cytoplasm of a cell to form a furrow that resembles a cleavage furrow but does not complete cytokinesis. References: PMID:10751167, PMID:30990821, PMID:7729583 Sources: GOC:mah Relationships: is a type of GO:0032501; BFO_0000050 embryo development [GO:0009790]